{
  "gene_name": "Testis-expressed protein 48",
  "gene_symbol": "TEX48",
  "term_label": "Unknown cellular component",
  "gene": "UniProtKB:A0A1B0GUV7",
  "term_id": "UNKNOWN:0003"
}